{
  "gene_name": "Guanylate-binding protein 2",
  "gene_symbol": "GBP2",
  "term_label": "cellular response to type II interferon",
  "term_id": "GO:0071346",
  "gene": "UniProtKB:P32456"
}